{
  "gene_symbol": "OXSR1",
  "gene": "UniProtKB:O95747",
  "term_label": "cytosol",
  "gene_name": "Serine_threonine-protein kinase OSR1",
  "term_id": "GO:0005829"
}